{
  "gene_symbol": "PDE2A",
  "term_id": "GO:0004115",
  "gene_name": "cGMP-dependent 3',5'-cyclic phosphodiesterase",
  "term_label": "3',5'-cyclic-AMP phosphodiesterase activity",
  "gene": "UniProtKB:O00408"
}